{
  "gene_name": "Zinc finger and BTB domain-containing protein 39",
  "term_id": "GO:0001817",
  "gene": "UniProtKB:O15060",
  "gene_symbol": "ZBTB39",
  "term_label": "regulation of cytokine production"
}